{
  "gene_name": "Proteasome subunit beta type-6",
  "gene_symbol": "PSMB6",
  "term_label": "proteasome-mediated ubiquitin-dependent protein catabolic process",
  "term_id": "GO:0043161",
  "gene": "UniProtKB:P28072"
}